{
  "term_id": "UNKNOWN:0003",
  "gene": "UniProtKB:Q9Y2I1",
  "gene_name": "Nischarin",
  "term_label": "Unknown cellular component",
  "gene_symbol": "NISCH"
}